melanosome transport [GO:0032402] (biological process) Sources: GOC:ln Definition: The directed movement of melanosomes into, out of or within a cell, or between cells, by means of some agent such as a transporter or pore. Relationships: is a type of melanosome localization [GO:0032400]; is_a establishment of melanosome localization [GO:0032401]; is a type of GO:0051904 Regulation: regulated by regulation of melanosome transport [GO:1902908]; negatively regulated by negative regulation of melanosome transport [GO:1902909]; positively regulated by positive regulation of melanosome transport [GO:1902910]